{
  "gene_symbol": "PEF1",
  "gene": "UniProtKB:Q9UBV8",
  "gene_name": "Peflin",
  "term_id": "GO:0048208",
  "term_label": "COPII vesicle coating"
}